negative regulation of acetylcholine biosynthetic process [GO:1905922] (biological process) References: PMID:20164328 Sources: GOC:TermGenie, GOC:aruk, GOC:bc, GO_REF:0000058 Relationships: is a type of GO:0009890; is a type of regulation of acetylcholine biosynthetic process [GO:1905921]; negatively regulates acetylcholine biosynthetic process [GO:0008292] Also known as: down regulation of acetylcholine anabolism, down regulation of acetylcholine biosynthesis, down regulation of acetylcholine biosynthetic process, down regulation of acetylcholine formation, down regulation of acetylcholine synthesis, down-regulation of acetylcholine anabolism, down-regulation of acetylcholine biosynthesis, down-regulation of acetylcholine biosynthetic process, down-regulation of acetylcholine formation, down-regulation of acetylcholine synthesis, downregulation of acetylcholine anabolism, downregulation of acetylcholine biosynthesis, downregulation of acetylcholine biosynthetic process, downregulation of acetylcholine formation, downregulation of acetylcholine synthesis, negative regulation of acetylcholine anabolism, negative regulation of acetylcholine biosynthesis, negative regulation of acetylcholine formation, negative regulation of acetylcholine synthesis, inhibition of acetylcholine anabolism, inhibition of acetylcholine biosynthesis, inhibition of acetylcholine biosynthetic process, inhibition of acetylcholine formation, inhibition of acetylcholine synthesis Definition: Any process that stops, prevents or reduces the frequency, rate or extent of acetylcholine biosynthetic process.